phloretin hydrolase activity [GO:0050180] (MF) Definition: Catalysis of the reaction: H2O + phloretin = H+ + phloretate + phloroglucinol. Also known as: lactase-phlorizin hydrolase, 2',4,4',6'-tetrahydroxydehydrochalcone 1,3,5-trihydroxybenzenehydrolase activity Sources: EC:3.7.1.4, RHEA:23396 Relationships: is a type of hydrolase activity, acting on acid carbon-carbon bonds, in ketonic substances [GO:0016823]